{
  "term_label": "endoplasmic reticulum",
  "gene_symbol": "SEZ6L",
  "term_id": "GO:0005783",
  "gene": "UniProtKB:Q9BYH1",
  "gene_name": "Seizure 6-like protein"
}